negative regulation of maltotetraose transport [GO:1900322] (biological process) Definition: Any process that stops, prevents or reduces the frequency, rate or extent of maltotetraose transport. Sources: GOC:TermGenie, GOC:mengo_curators Also known as: down regulation of maltotetraose transport, down-regulation of maltotetraose transport, downregulation of maltotetraose transport, inhibition of maltotetraose transport Relationships: is a type of negative regulation of transport [GO:0051051]; is a type of regulation of maltotetraose transport [GO:1900321]; negatively regulates maltotetraose transport [GO:2001099]